alpha7-beta1 integrin-CD151 complex [GO:0071060] (cellular component) Definition: A protein complex that consists of an alpha7-beta1 integrin complex bound to the tetraspanin CD151. Also known as: ITGA7-ITGB1-CD151 complex Relationships: is a type of plasma membrane protein complex [GO:0098797] References: PMID:11884516